{
  "term_label": "neuron projection development",
  "gene": "UniProtKB:Q99748",
  "gene_name": "Neurturin",
  "term_id": "GO:0031175",
  "gene_symbol": "NRTN"
}